digestive tract development [GO:0048565] (biological process) Definition: The process whose specific outcome is the progression of the digestive tract over time, from its formation to the mature structure. The digestive tract is the anatomical structure through which food passes and is processed. Also known as: gut development, intestinal development, intestine development Sources: GOC:go_curators Relationships: is a type of tube development [GO:0035295]; is part of digestive system development [GO:0055123] Subtypes: midgut development [GO:0007494], embryonic digestive tract development [GO:0048566], hindgut development [GO:0061525]